{
  "term_id": "UNKNOWN:0001",
  "gene": "UniProtKB:Q9Y3C7",
  "term_label": "Unknown molecular function",
  "gene_name": "Mediator of RNA polymerase II transcription subunit 31",
  "gene_symbol": "MED31"
}